{
  "term_id": "GO:0005634",
  "term_label": "nucleus",
  "gene_name": "Zinc finger protein 578",
  "gene": "UniProtKB:Q96N58",
  "gene_symbol": "ZNF578"
}